abscisic acid catabolic process [GO:0046345] (biological process) Definition: The chemical reactions and pathways resulting in the breakdown of abscisic acid, 5-(1-hydroxy-2,6,6,trimethyl-4-oxocyclohex-2-en-1-y1)-3-methylpenta-2,4-dienoic acid. Also known as: abscisic acid breakdown, abscisic acid catabolism, abscisic acid degradation Sources: GOC:ai Relationships: is a type of GO:0009687; is a type of sesquiterpenoid catabolic process [GO:0016107]; is a type of apocarotenoid catabolic process [GO:0043290]; is a type of GO:0046164; is a type of monocarboxylic acid catabolic process [GO:0072329]; is a type of GO:0120256